{
  "term_label": "proteolysis",
  "term_id": "GO:0006508",
  "gene": "UniProtKB:Q86TI2",
  "gene_name": "Dipeptidyl peptidase 9",
  "gene_symbol": "DPP9"
}